{
  "term_id": "UNKNOWN:0002",
  "gene_name": "Echinoderm microtubule-associated protein-like 6",
  "gene_symbol": "EML6",
  "gene": "UniProtKB:Q6ZMW3",
  "term_label": "Unknown biological process"
}